{
  "term_label": "endoplasmic reticulum",
  "gene": "UniProtKB:Q5BJF2",
  "gene_name": "Sigma intracellular receptor 2",
  "term_id": "GO:0005783",
  "gene_symbol": "TMEM97"
}